{
  "gene": "UniProtKB:Q7Z2H8",
  "term_id": "GO:0015180",
  "gene_name": "Proton-coupled amino acid transporter 1",
  "gene_symbol": "SLC36A1",
  "term_label": "L-alanine transmembrane transporter activity"
}